{
  "gene_symbol": "TUBE1",
  "gene_name": "Tubulin epsilon chain",
  "gene": "UniProtKB:Q9UJT0",
  "term_id": "GO:0005737",
  "term_label": "cytoplasm"
}